heptadecane biosynthetic process [GO:1900636] (biological process) Sources: GOC:TermGenie, GOC:mengo_curators Relationships: is a type of alkane biosynthetic process [GO:0043447]; is a type of heptadecane metabolic process [GO:1900635] Also known as: heptadecane anabolism, heptadecane biosynthesis, heptadecane formation, heptadecane synthesis Definition: The chemical reactions and pathways resulting in the formation of heptadecane. Regulation: RO_0002211 by regulation of heptadecane biosynthetic process [GO:1900896]; negatively regulated by negative regulation of heptadecane biosynthetic process [GO:1900897]; positively regulated by positive regulation of heptadecane biosynthetic process [GO:1900898]